{
  "gene_name": "Histone-lysine N-methyltransferase PRDM16",
  "term_id": "GO:0000978",
  "gene_symbol": "PRDM16",
  "gene": "UniProtKB:Q9HAZ2",
  "term_label": "RNA polymerase II cis-regulatory region sequence-specific DNA binding"
}